{
  "gene_name": "Structural maintenance of chromosomes protein 1B",
  "term_id": "GO:0005634",
  "term_label": "nucleus",
  "gene_symbol": "SMC1B",
  "gene": "UniProtKB:Q8NDV3"
}